{
  "term_id": "UNKNOWN:0001",
  "term_label": "Unknown molecular function",
  "gene_symbol": "A0A5F9ZHU2",
  "gene_name": "Uncharacterized protein",
  "gene": "UniProtKB:A0A5F9ZHU2"
}